{
  "gene": "UniProtKB:Q16659",
  "gene_symbol": "MAPK6",
  "term_id": "GO:0005634",
  "term_label": "nucleus",
  "gene_name": "Mitogen-activated protein kinase 6"
}